{
  "term_id": "GO:0038187",
  "gene_name": "Asialoglycoprotein receptor 2",
  "gene_symbol": "ASGR2",
  "term_label": "pattern recognition receptor activity",
  "gene": "UniProtKB:P07307"
}